positive regulation of oxytocin production [GO:0140668] (biological process) Definition: Any process that activates or increases the frequency, rate or extent of production of oxytocin. References: PMID:25096581 Relationships: is a type of positive regulation of gene expression [GO:0010628]; is a type of GO:0140667; positively regulates oxytocin production [GO:0036162]